{
  "term_id": "GO:0090336",
  "gene_name": "Fibronectin type III domain-containing protein 5",
  "gene": "UniProtKB:Q8NAU1",
  "term_label": "positive regulation of brown fat cell differentiation",
  "gene_symbol": "FNDC5"
}